{
  "term_label": "morphogenesis of an epithelium",
  "gene": "UniProtKB:Q04695",
  "gene_symbol": "KRT17",
  "term_id": "GO:0002009",
  "gene_name": "Keratin, type I cytoskeletal 17"
}